{
  "term_label": "trans-Golgi network",
  "gene_symbol": "KLHL20",
  "gene_name": "Kelch-like protein 20",
  "gene": "UniProtKB:Q9Y2M5",
  "term_id": "GO:0005802"
}